{
  "gene_symbol": "RAB25",
  "gene_name": "Ras-related protein Rab-25",
  "gene": "UniProtKB:P57735",
  "term_label": "exocytosis",
  "term_id": "GO:0006887"
}